{
  "term_id": "UNKNOWN:0003",
  "gene_symbol": "TRGC1",
  "gene": "UniProtKB:P0CF51",
  "gene_name": "T cell receptor gamma constant 1",
  "term_label": "Unknown cellular component"
}